{
  "gene": "UniProtKB:Q6UVK1",
  "gene_name": "Chondroitin sulfate proteoglycan 4",
  "gene_symbol": "CSPG4",
  "term_id": "GO:0007165",
  "term_label": "signal transduction"
}